{
  "term_id": "UNKNOWN:0001",
  "gene": "UniProtKB:Q6EKJ0",
  "gene_name": "General transcription factor II-I repeat domain-containing protein 2B",
  "gene_symbol": "GTF2IRD2B",
  "term_label": "Unknown molecular function"
}